regulation of meiotic nuclear division [GO:0040020] (biological process) Subtypes: negative regulation of meiotic nuclear division [GO:0045835], GO:0045836, regulation of meiosis I [GO:0060631] Also known as: regulation of meiosis Relationships: is_a regulation of cell cycle process [GO:0010564]; is a type of GO:0051445; is a type of regulation of nuclear division [GO:0051783]; regulates meiotic nuclear division [GO:0140013] Definition: Any process that modulates the frequency, rate or extent of meiotic nuclear division, the process in which the nucleus of a diploid cell divides twice forming four haploid cells, one or more of which usually function as gametes. Sources: GOC:ems, GOC:ma